{
  "term_label": "vesicle-mediated transport",
  "gene_symbol": "SYT13",
  "gene_name": "Synaptotagmin-13",
  "term_id": "GO:0016192",
  "gene": "UniProtKB:Q7L8C5"
}